exo-poly-alpha-galacturonosidase activity [GO:0033917] (molecular function) Relationships: is a type of hydrolase activity, hydrolyzing O-glycosyl compounds [GO:0004553] Also known as: exopolygalacturanosidase activity, exopolygalacturonosidase activity Sources: EC:3.2.1.82 Definition: Catalysis of the hydrolysis of pectic acid from the non-reducing end, releasing digalacturonate.